{
  "gene": "UniProtKB:Q13634",
  "term_label": "calcium-dependent cell-cell adhesion",
  "gene_name": "Cadherin-18",
  "gene_symbol": "CDH18",
  "term_id": "GO:0016339"
}